CENP-A recruiting complex [GO:0098654] (cellular component) References: PMID:24774534 Definition: A protein complex that includes Mis16(Yippee family) and/or Mis18 (WD repeat) subunits that is involved in the deposition of centromere specific (CENP-A containing) nucleosomes at the centromere. Relationships: is a type of GO:0140513 Also known as: MIS18 complex